{
  "gene_name": "Atlastin-3",
  "term_label": "GTPase activity",
  "gene_symbol": "ATL3",
  "term_id": "GO:0003924",
  "gene": "UniProtKB:Q6DD88"
}